{
  "term_label": "mRNA binding",
  "gene_name": "Serine_arginine-rich splicing factor 5",
  "gene": "UniProtKB:Q13243",
  "term_id": "GO:0003729",
  "gene_symbol": "SRSF5"
}